{
  "gene_symbol": "TSNAXIP1",
  "gene_name": "Translin-associated factor X-interacting protein 1",
  "gene": "UniProtKB:Q2TAA8",
  "term_id": "UNKNOWN:0002",
  "term_label": "Unknown biological process"
}